{
  "gene_name": "Homeobox protein Hox-B6",
  "gene": "UniProtKB:P17509",
  "gene_symbol": "HOXB6",
  "term_label": "nucleus",
  "term_id": "GO:0005634"
}